{
  "gene_name": "Tolloid-like protein 1",
  "term_label": "metalloendopeptidase activity",
  "term_id": "GO:0004222",
  "gene": "UniProtKB:O43897",
  "gene_symbol": "TLL1"
}